spliceosomal complex [GO:0005681] (cellular component) Subtypes: U2-type spliceosomal complex [GO:0005684], U12-type spliceosomal complex [GO:0005689], GO:0044530, prespliceosome [GO:0071010], precatalytic spliceosome [GO:0071011], catalytic step 1 spliceosome [GO:0071012], catalytic step 2 spliceosome [GO:0071013], post-mRNA release spliceosomal complex [GO:0071014], post-spliceosomal complex [GO:0071020], trans spliceosomal complex [GO:0071023] References: PMID:19239890 Sources: GOC:editors, GOC:mah, ISBN:0198547684 Definition: Any of a series of ribonucleoprotein complexes that contain snRNA(s) and small nuclear ribonucleoproteins (snRNPs), and are formed sequentially during the spliceosomal splicing of one or more substrate RNAs, and which also contain the RNA substrate(s) from the initial target RNAs of splicing, the splicing intermediate RNA(s), to the final RNA products. During cis-splicing, the initial target RNA is a single, contiguous RNA transcript, whether mRNA, snoRNA, etc., and the released products are a spliced RNA and an excised intron, generally as a lariat structure. During trans-splicing, there are two initial substrate RNAs, the spliced leader RNA and a pre-mRNA. Relationships: is a type of nuclear protein-containing complex [GO:0140513]; is a type of GO:1990904 Also known as: spliceosome, spliceosome complex